{
  "term_label": "cytosolic small ribosomal subunit",
  "gene_name": "Small ribosomal subunit protein uS10",
  "gene_symbol": "RPS20",
  "term_id": "GO:0022627",
  "gene": "UniProtKB:P60866"
}